{
  "gene": "UniProtKB:Q5H9J9",
  "gene_symbol": "TCP11X2",
  "term_id": "GO:1902490",
  "term_label": "regulation of sperm capacitation",
  "gene_name": "T-complex protein 11 X-linked protein 2"
}